{
  "term_id": "GO:0046329",
  "gene_name": "Kelch-like protein 31",
  "term_label": "negative regulation of JNK cascade",
  "gene": "UniProtKB:Q9H511",
  "gene_symbol": "KLHL31"
}